{
  "gene": "UniProtKB:Q8IZ52",
  "term_label": "chondroitin sulfate proteoglycan biosynthetic process",
  "term_id": "GO:0050650",
  "gene_name": "Chondroitin sulfate synthase 2",
  "gene_symbol": "CHPF"
}